{
  "gene_name": "Deoxyribose-phosphate aldolase",
  "term_id": "UNKNOWN:0003",
  "gene_symbol": "DERA",
  "gene": "UniProtKB:Q9Y315",
  "term_label": "Unknown cellular component"
}